leukemia inhibitory factor receptor activity [GO:0004923] (molecular function) Definition: Combining with leukemia inhibitory factor (LIF) and transmitting the signal from one side of the membrane to the other to initiate a change in cell activity. Also known as: LIF receptor activity, leukemia inhibitory factor receptor beta-protein activity Sources: GOC:bf, GOC:mah, GOC:signaling Relationships: is a type of ciliary neurotrophic factor receptor activity [GO:0004897]; is part of leukemia inhibitory factor signaling pathway [GO:0048861]